{
  "term_id": "GO:0019722",
  "gene": "UniProtKB:O00421",
  "term_label": "calcium-mediated signaling",
  "gene_name": "C-C chemokine receptor-like 2",
  "gene_symbol": "CCRL2"
}